{
  "term_label": "G protein-coupled receptor activity",
  "term_id": "GO:0004930",
  "gene_name": "Prokineticin receptor 2",
  "gene": "UniProtKB:Q8NFJ6",
  "gene_symbol": "PROKR2"
}